{
  "term_label": "nucleus",
  "gene_name": "G1_S-specific cyclin-E1",
  "gene_symbol": "CCNE1",
  "term_id": "GO:0005634",
  "gene": "UniProtKB:P24864"
}